{
  "term_label": "Unknown cellular component",
  "gene_symbol": "A0A8V8TPC4",
  "gene_name": "Uncharacterized protein",
  "gene": "UniProtKB:A0A8V8TPC4",
  "term_id": "UNKNOWN:0003"
}